achromobactin catabolic process [GO:0042862] (biological process) Relationships: is_a amide metabolic process [GO:0043603]; is a type of siderophore catabolic process [GO:0046215]; is a type of carboxylic acid catabolic process [GO:0046395] Also known as: achromobactin breakdown, achromobactin catabolism, achromobactin degradation Definition: The chemical reactions and pathways resulting in the breakdown of achromobactin, a citrate siderophore. References: PMID:10928541 Sources: GOC:jl